{
  "term_label": "meiotic chromosome condensation",
  "gene": "UniProtKB:Q6IBW4",
  "term_id": "GO:0010032",
  "gene_name": "Condensin-2 complex subunit H2",
  "gene_symbol": "NCAPH2"
}